{
  "term_label": "protein transport to vacuole involved in ubiquitin-dependent protein catabolic process via the multivesicular body sorting pathway",
  "gene_symbol": "SNF8",
  "gene_name": "Vacuolar-sorting protein SNF8",
  "gene": "UniProtKB:Q96H20",
  "term_id": "GO:0043328"
}